{
  "gene": "UniProtKB:Q9BYR5",
  "gene_symbol": "KRTAP4-2",
  "gene_name": "Keratin-associated protein 4-2",
  "term_id": "UNKNOWN:0003",
  "term_label": "Unknown cellular component"
}